atrichoblast fate specification [GO:0010056] (biological process) Regulation: regulated by GO:0010058; positively regulated by positive regulation of atrichoblast fate specification [GO:0010059]; negatively regulated by negative regulation of atrichoblast fate specification [GO:0010060] Sources: GOC:tb Definition: The process involved in the specification of an atrichoblast. Relationships: is a type of GO:0090628; is part of atrichoblast differentiation [GO:0010055]